{
  "gene_symbol": "CRISP3",
  "term_id": "GO:0005615",
  "gene": "UniProtKB:P54108",
  "gene_name": "Cysteine-rich secretory protein 3",
  "term_label": "extracellular space"
}